host cell endoplasmic reticulum membrane [GO:0044167] (CC) Also known as: host endoplasmic reticulum membrane Definition: The lipid bilayer surrounding the host cell endoplasmic reticulum. Relationships: is a type of host cell membrane [GO:0033644]; is part of host cell endomembrane system [GO:0033645]; BFO_0000050 host cell endoplasmic reticulum [GO:0044165] Subtypes: GO:0044169, host cell smooth endoplasmic reticulum membrane [GO:0044171] Sources: GOC:jl